{
  "gene_name": "Fibroblast growth factor 5",
  "term_id": "GO:0008083",
  "gene_symbol": "FGF5",
  "gene": "UniProtKB:P12034",
  "term_label": "growth factor activity"
}